{
  "term_label": "glycerol-3-phosphate dehydrogenase (quinone) activity",
  "gene_symbol": "GPD2",
  "gene_name": "Glycerol-3-phosphate dehydrogenase, mitochondrial",
  "term_id": "GO:0004368",
  "gene": "UniProtKB:P43304"
}